{
  "gene": "UniProtKB:Q86Y39",
  "term_label": "Unknown biological process",
  "gene_name": "NADH dehydrogenase [ubiquinone] 1 alpha subcomplex subunit 11",
  "gene_symbol": "NDUFA11",
  "term_id": "UNKNOWN:0002"
}